DnaA-DiaA complex [GO:1990102] (cellular component) Definition: A protein-DNA complex containing a tetramer of DiaA attached to multiple DnaA molecule bound to oriC DNA. Regulates timely initiation of chromosomal replication during the cell cycle by stimulating assembly of DnaA-oriC complexes, conformational changes in ATP-DnaA initiation complexes, and unwinding of oriC duplex DNA. References: PMID:15326179, PMID:17699754 Sources: GOC:bhm Also known as: DnaA-DiaA-DNA complex Relationships: is a type of primosome complex [GO:1990077]; has part DnaA-oriC complex [GO:1990101]; has part DiaA complex [GO:1990125]